{
  "gene_name": "Trafficking kinesin-binding protein 2",
  "term_label": "protein targeting",
  "gene_symbol": "TRAK2",
  "term_id": "GO:0006605",
  "gene": "UniProtKB:O60296"
}